{
  "term_id": "GO:0005829",
  "gene_name": "MIF4G domain-containing protein",
  "term_label": "cytosol",
  "gene_symbol": "MIF4GD",
  "gene": "UniProtKB:A9UHW6"
}